{
  "gene": "UniProtKB:Q502X0",
  "gene_symbol": "MORN2",
  "gene_name": "MORN repeat-containing protein 2",
  "term_label": "Unknown cellular component",
  "term_id": "UNKNOWN:0003"
}